{
  "term_label": "plasma membrane",
  "gene": "UniProtKB:Q9NYG8",
  "gene_name": "Potassium channel subfamily K member 4",
  "term_id": "GO:0005886",
  "gene_symbol": "KCNK4"
}